{
  "gene_name": "Eukaryotic translation initiation factor 3 subunit K",
  "term_id": "GO:0005852",
  "gene_symbol": "EIF3K",
  "gene": "UniProtKB:Q9UBQ5",
  "term_label": "eukaryotic translation initiation factor 3 complex"
}